{
  "gene": "UniProtKB:O15540",
  "gene_symbol": "FABP7",
  "gene_name": "Fatty acid-binding protein, brain",
  "term_id": "GO:0005504",
  "term_label": "fatty acid binding"
}